caffeoyl-CoA O-methyltransferase activity [GO:0042409] (molecular function) Definition: Catalysis of the reaction: S-adenosyl-L-methionine + caffeoyl-CoA = S-adenosyl-L-homocysteine + feruloyl-CoA. Relationships: is a type of O-methyltransferase activity [GO:0008171]; is_a GO:0008757 Sources: EC:2.1.1.104 Also known as: caffeoyl CoA:S-adenosyl-L-methionine O-methyltransferase activity, caffeoyl coenzyme A methyltransferase activity, caffeoyl-CoA 3-O-methyltransferase activity, S-adenosyl-L-methionine:caffeoyl-CoA 3-O-methyltransferase activity, trans-caffeoyl-CoA 3-O-methyltransferase activity